{
  "gene_name": "Patatin-like phospholipase domain-containing protein 7",
  "term_id": "GO:0005783",
  "term_label": "endoplasmic reticulum",
  "gene_symbol": "PNPLA7",
  "gene": "UniProtKB:Q6ZV29"
}